{
  "gene_symbol": "ABHD5",
  "gene_name": "1-acylglycerol-3-phosphate O-acyltransferase ABHD5",
  "gene": "UniProtKB:Q8WTS1",
  "term_id": "GO:0006654",
  "term_label": "phosphatidic acid biosynthetic process"
}